{
  "term_id": "GO:0019722",
  "term_label": "calcium-mediated signaling",
  "gene": "UniProtKB:P46092",
  "gene_name": "C-C chemokine receptor type 10",
  "gene_symbol": "CCR10"
}